host-mediated perturbation of symbiont process [GO:0051851] (biological process) Subtypes: host-mediated perturbation of viral process [GO:0044788], host-mediated suppression of symbiont invasion [GO:0046597], host-mediated modulation of intestinal microbiota composition [GO:0048874], host-mediated modulation of oral microbiota composition [GO:0120332] Definition: The process in which an host alters or subverts a process in a symbiont organism. The symbiont is defined as the smaller of the organisms involved in a symbiotic interaction. Also known as: modulation by host of symbiont process, modification by host of symbiont morphology or physiology Sources: GOC:cc Relationships: is a type of GO:0035821